{
  "term_label": "BLOC-3 complex",
  "gene_name": "BLOC-3 complex member HPS1",
  "gene": "UniProtKB:Q92902",
  "gene_symbol": "HPS1",
  "term_id": "GO:0031085"
}